dichloromethane dehalogenase activity [GO:0018834] (molecular function) Also known as: dichloromethane chloride-lyase (adding H2O; chloride-hydrolysing; formaldehyde-forming), dichloromethane chloride-lyase (chloride-hydrolysing) Sources: EC:4.5.1.3, RHEA:15397 Definition: Catalysis of the reaction: dichloromethane + H2O = 2 chloride + formaldehyde + 2 H+. Relationships: is a type of carbon-halide lyase activity [GO:0016848]